{
  "gene_symbol": "RS1",
  "gene": "UniProtKB:O15537",
  "term_id": "GO:0010842",
  "gene_name": "Retinoschisin",
  "term_label": "retina layer formation"
}